calcium-dependent activation of synaptic vesicle fusion [GO:0099502] (BP) Regulation: regulated by GO:0150037 Definition: The regulatory process by which increased cytosolic calcium levels lead to the the fusion of synaptic vesicles with the presynaptic active zone membrane by bringing primed synaptic vesicle membrane into contact with membrane presynaptic active zone membrane. References: PMID:23060190 Relationships: is a type of GO:0031632; is part of synaptic vesicle exocytosis [GO:0016079]